{
  "term_label": "RNA polymerase II cis-regulatory region sequence-specific DNA binding",
  "gene": "UniProtKB:Q9BX82",
  "term_id": "GO:0000978",
  "gene_symbol": "ZNF471",
  "gene_name": "Zinc finger protein 471"
}